response to Gram-positive bacterium [GO:0140459] (biological process) Relationships: is a type of GO:0009617 References: PMID:23664307 Definition: Any process that results in a change in state or activity of a cell or an organism (in terms of movement, secretion, enzyme production, gene expression, etc.) as a result of a stimulus from a Gram-positive bacterium.